{
  "gene_symbol": "ZNF777",
  "gene": "UniProtKB:Q9ULD5",
  "term_label": "regulation of transcription by RNA polymerase II",
  "gene_name": "Zinc finger protein 777",
  "term_id": "GO:0006357"
}